{
  "gene": "UniProtKB:Q8NGJ1",
  "term_label": "plasma membrane",
  "term_id": "GO:0005886",
  "gene_name": "Olfactory receptor 4D6",
  "gene_symbol": "OR4D6"
}